protein polyubiquitination [GO:0000209] (biological process) References: PMID:26906419 Subtypes: protein K29-linked ubiquitination [GO:0035519], GO:0044314, protein K63-linked ubiquitination [GO:0070534], protein K48-linked ubiquitination [GO:0070936], protein K11-linked ubiquitination [GO:0070979], protein K6-linked ubiquitination [GO:0085020], GO:0097039, GO:0141198, protein K33-linked ubiquitination [GO:1990390] Definition: Addition of multiple ubiquitin groups to a protein, forming a ubiquitin chain. Relationships: is a type of protein ubiquitination [GO:0016567] Regulation: regulated by GO:1902914; negatively regulated by negative regulation of protein polyubiquitination [GO:1902915]; RO_0002213 by GO:1902916 Also known as: protein polyubiquitinylation, protein polyubiquitylation, polyubiquitin